{
  "gene_symbol": "TNKS1BP1",
  "gene_name": "182 kDa tankyrase-1-binding protein",
  "gene": "UniProtKB:Q9C0C2",
  "term_id": "GO:0071479",
  "term_label": "cellular response to ionizing radiation"
}